{
  "term_id": "GO:0019882",
  "gene_symbol": "CD74",
  "gene": "UniProtKB:P04233",
  "gene_name": "HLA class II histocompatibility antigen gamma chain",
  "term_label": "antigen processing and presentation"
}